{
  "term_id": "UNKNOWN:0001",
  "gene_name": "Putative uncharacterized protein encoded by LINC00304",
  "gene": "UniProtKB:Q8N9R0",
  "gene_symbol": "LINC00304",
  "term_label": "Unknown molecular function"
}